{
  "term_label": "double-strand break repair",
  "gene_name": "Serine-protein kinase ATM",
  "term_id": "GO:0006302",
  "gene": "UniProtKB:Q13315",
  "gene_symbol": "ATM"
}